{
  "gene_symbol": "MAPKBP1",
  "gene": "UniProtKB:O60336",
  "term_label": "cytoplasm",
  "gene_name": "Mitogen-activated protein kinase-binding protein 1",
  "term_id": "GO:0005737"
}